{
  "term_label": "Unknown cellular component",
  "gene_name": "SH2 domain-containing adapter protein B",
  "term_id": "UNKNOWN:0003",
  "gene_symbol": "SHB",
  "gene": "UniProtKB:Q15464"
}